cyclin-dependent protein kinase holoenzyme complex [GO:0000307] (cellular component) Definition: Cyclin-dependent protein kinases (CDKs) are enzyme complexes that contain a kinase catalytic subunit associated with a regulatory cyclin partner. References: PMID:11602261 Sources: GOC:krc Also known as: CDK holoenzyme Relationships: is a type of serine/threonine protein kinase complex [GO:1902554] Subtypes: cytoplasmic cyclin-dependent protein kinase holoenzyme complex [GO:0000308], cyclin K-CDK12 complex [GO:0002944], GO:0002945, GO:0019908, MPF complex [GO:0031387], cyclin A1-CDK1 complex [GO:0097121], cyclin A2-CDK1 complex [GO:0097122], cyclin A1-CDK2 complex [GO:0097123], cyclin A2-CDK2 complex [GO:0097124], cyclin B1-CDK1 complex [GO:0097125], cyclin B2-CDK1 complex [GO:0097126], cyclin B3-CDK2 complex [GO:0097127], cyclin D1-CDK4 complex [GO:0097128], cyclin D2-CDK4 complex [GO:0097129], cyclin D3-CDK4 complex [GO:0097130], cyclin D1-CDK6 complex [GO:0097131], cyclin D2-CDK6 complex [GO:0097132], GO:0097133, cyclin E1-CDK2 complex [GO:0097134], cyclin E2-CDK2 complex [GO:0097135], cyclin L-CDK11 complex [GO:0180038], Pho85-Pho80 CDK-cyclin complex [GO:1990860]